{
  "term_id": "GO:0071818",
  "gene_name": "Large proline-rich protein BAG6",
  "gene": "UniProtKB:P46379",
  "term_label": "BAT3 complex",
  "gene_symbol": "BAG6"
}